{
  "gene": "UniProtKB:P59051",
  "gene_symbol": "BRWD1-AS2",
  "term_id": "UNKNOWN:0001",
  "gene_name": "Putative uncharacterized protein encoded by BRWD1-AS2",
  "term_label": "Unknown molecular function"
}